{
  "term_id": "GO:0006099",
  "gene_symbol": "OGDH",
  "gene": "UniProtKB:Q02218",
  "term_label": "tricarboxylic acid cycle",
  "gene_name": "2-oxoglutarate dehydrogenase complex component E1"
}